glomerular mesangial cell proliferation [GO:0072110] (biological process) Sources: GOC:mtg_kidney_jan10 Definition: The multiplication or reproduction of glomerular mesangial cells, resulting in the expansion of the population. Regulation: regulated by regulation of glomerular mesangial cell proliferation [GO:0072124]; negatively regulated by GO:0072125; positively regulated by positive regulation of glomerular mesangial cell proliferation [GO:0072126] Subtypes: mesonephric glomerular mesangial cell proliferation involved in mesonephros development [GO:0061269], intraglomerular mesangial cell proliferation [GO:0072123], metanephric glomerular mesangial cell proliferation involved in metanephros development [GO:0072262] Relationships: is a type of cell proliferation involved in kidney development [GO:0072111]; is part of GO:0072109